{
  "gene_name": "Membrane-spanning 4-domains subfamily A member 18",
  "gene": "UniProtKB:Q3C1V0",
  "term_label": "Unknown molecular function",
  "term_id": "UNKNOWN:0001",
  "gene_symbol": "MS4A18"
}